{
  "term_id": "UNKNOWN:0002",
  "gene": "UniProtKB:B7Z8K6",
  "term_label": "Unknown biological process",
  "gene_symbol": "TRDC",
  "gene_name": "T cell receptor delta constant"
}